{
  "gene_name": "Intraflagellar transport protein 20 homolog",
  "gene_symbol": "IFT20",
  "gene": "UniProtKB:Q8IY31",
  "term_label": "non-motile cilium",
  "term_id": "GO:0097730"
}